{
  "term_id": "GO:0007186",
  "term_label": "G protein-coupled receptor signaling pathway",
  "gene_symbol": "F2RL3",
  "gene_name": "Proteinase-activated receptor 4",
  "gene": "UniProtKB:Q96RI0"
}